{
  "gene": "UniProtKB:O60609",
  "term_id": "GO:0009897",
  "term_label": "external side of plasma membrane",
  "gene_name": "GDNF family receptor alpha-3",
  "gene_symbol": "GFRA3"
}